zymogen inhibition [GO:0097341] (biological process) Definition: Any process that prevents the proteolytic processing of an inactive enzyme to an active form. References: PMID:20383739 Sources: GOC:mtg_apoptosis Also known as: prevention of zymogen activation Relationships: is a type of negative regulation of protein processing [GO:0010955]